cerebellar Purkinje cell layer morphogenesis [GO:0021692] (biological process) Relationships: is a type of anatomical structure morphogenesis [GO:0009653]; is part of cerebellar Purkinje cell layer development [GO:0021680]; is part of cerebellar cortex morphogenesis [GO:0021696] Definition: The process in which the anatomical structure of the cerebellar Purkinje cell layer is generated and organized. The Purkinje cell layer lies just underneath the molecular layer of the cerebellar cortex. It contains the neuronal cell bodies of the Purkinje cells that are arranged side by side in a single layer. Candelabrum interneurons are vertically oriented between the Purkinje cells. Purkinje neurons are inhibitory and provide the output of the cerebellar cortex through axons that project into the white matter. Extensive dendritic trees from the Purkinje cells extend upward in a single plane into the molecular layer where they synapse with parallel fibers of granule cells. Sources: GOC:cls, GOC:dgh, GOC:dph, GOC:jid, GO_REF:0000021